{
  "gene": "UniProtKB:Q8TD06",
  "gene_name": "Anterior gradient protein 3",
  "term_id": "GO:0005783",
  "term_label": "endoplasmic reticulum",
  "gene_symbol": "AGR3"
}